{
  "gene_name": "NLR family CARD domain-containing protein 3",
  "gene": "UniProtKB:Q7RTR2",
  "gene_symbol": "NLRC3",
  "term_label": "cytosol",
  "term_id": "GO:0005829"
}